{
  "gene_symbol": "ARHGAP35",
  "term_id": "GO:0005829",
  "term_label": "cytosol",
  "gene_name": "Rho GTPase-activating protein 35",
  "gene": "UniProtKB:Q9NRY4"
}